{
  "term_id": "GO:0033130",
  "term_label": "acetylcholine receptor binding",
  "gene": "UniProtKB:Q13702",
  "gene_symbol": "RAPSN",
  "gene_name": "43 kDa receptor-associated protein of the synapse"
}